{
  "term_id": "GO:0008117",
  "term_label": "sphinganine-1-phosphate aldolase activity",
  "gene": "UniProtKB:O95470",
  "gene_symbol": "SGPL1",
  "gene_name": "Sphingosine-1-phosphate lyase 1"
}